quaternary ammonium group binding [GO:0050997] (MF) Also known as: quaternary amine binding Sources: GOC:ai Definition: Binding to a quaternary ammonium group, including glycine betaine, choline, carnitine and proline. A quaternary ammonium group is any compound that can be regarded as derived from ammonium hydroxide or an ammonium salt by replacement of all four hydrogen atoms of the NH4+ ion by organic groups. Relationships: is a type of small molecule binding [GO:0036094] Subtypes: thiamine pyrophosphate binding [GO:0030976], phosphatidylcholine binding [GO:0031210], hydroxyectoine binding [GO:0033295]